{
  "term_id": "GO:0005886",
  "term_label": "plasma membrane",
  "gene_symbol": "MYO1H",
  "gene": "UniProtKB:Q8N1T3",
  "gene_name": "Unconventional myosin-Ih"
}